{
  "gene_symbol": "UBE2D3",
  "gene_name": "Ubiquitin-conjugating enzyme E2 D3",
  "term_id": "GO:0061631",
  "gene": "UniProtKB:P61077",
  "term_label": "ubiquitin conjugating enzyme activity"
}